negative regulation of progesterone secretion [GO:2000871] (biological process) Relationships: is a type of negative regulation of female gonad development [GO:2000195]; is a type of negative regulation of steroid hormone secretion [GO:2000832]; is_a GO:2000870; negatively regulates progesterone secretion [GO:0042701] Sources: GOC:sl Definition: Any process that stops, prevents or reduces the frequency, rate or extent of progesterone secretion.